pyrimidine ribonucleotide catabolic process [GO:0009222] (biological process) Definition: The chemical reactions and pathways resulting in the breakdown of a pyrimidine ribonucleotide, a compound consisting of nucleoside (a pyrimidine base linked to a ribose sugar) esterified with a phosphate group at either the 3' or 5'-hydroxyl group of the sugar. Subtypes: GO:0006245, GO:0006248, CTP catabolic process [GO:0006254], UDP catabolic process [GO:0006256], GO:0046045, TTP catabolic process [GO:0046047], GO:0046050, UTP catabolic process [GO:0046052], CDP catabolic process [GO:0046706] Relationships: is a type of pyrimidine nucleotide catabolic process [GO:0006244]; is a type of pyrimidine ribonucleotide metabolic process [GO:0009218]; is a type of ribonucleotide catabolic process [GO:0009261] Also known as: pyrimidine ribonucleotide breakdown, pyrimidine ribonucleotide catabolism, pyrimidine ribonucleotide degradation Sources: GOC:go_curators, ISBN:0198506732